curli assembly [GO:0098775] (biological process) Definition: The process of assembly of curli, extracellular fibers produced by enteric bacteria. This process occurs outside the cell, where it is coupled to secretion across the cell outer membrane via nucleation by elements of the transporter complex. References: PMID:16704339 Relationships: is a type of GO:0009297